{
  "gene_name": "Lamin-B1",
  "term_id": "GO:0006998",
  "term_label": "nuclear envelope organization",
  "gene_symbol": "LMNB1",
  "gene": "UniProtKB:P20700"
}